{
  "term_id": "GO:0005730",
  "gene_symbol": "RBIS",
  "gene_name": "Ribosomal biogenesis factor",
  "term_label": "nucleolus",
  "gene": "UniProtKB:Q8N0T1"
}